histamine oxidase activity [GO:0052598] (MF) Relationships: is a type of diamine oxidase activity [GO:0052597] Also known as: 1H-Imidazole-4-ethanamine oxidase activity, 1H-Imidazole-4-ethanamine:oxygen oxidoreductase (deaminating) activity, histamine:oxygen oxidoreductase (deaminating) activity Sources: RHEA:25625 Definition: Catalysis of the reaction: H2O + histamine + O2 = H2O2 + imidazole-4-acetaldehyde + NH4+.